{
  "gene_symbol": "FOXO3",
  "gene": "UniProtKB:O43524",
  "term_label": "response to starvation",
  "term_id": "GO:0042594",
  "gene_name": "Forkhead box protein O3"
}